galactose:proton symporter activity [GO:0015517] (molecular function) Definition: Enables the transfer of a solute or solutes from one side of a membrane to the other according to the reaction: galactose(out) + H+(out) = galactose(in) + H+(in). Also known as: lactose, galactose:hydrogen symporter activity, galactose:hydrogen symporter activity Relationships: is a type of GO:0005354; is a type of hexose:proton symporter activity [GO:0009679] Sources: TC:2.A.1.1.1, TC:2.A.1.1.9